{
  "term_id": "GO:0005634",
  "term_label": "nucleus",
  "gene": "UniProtKB:Q7Z309",
  "gene_name": "PABIR family member 2",
  "gene_symbol": "PABIR2"
}